regulation of neutrophil mediated killing of gram-positive bacterium [GO:0070952] (biological process) Relationships: is a type of GO:0070950; regulates neutrophil-mediated killing of gram-positive bacterium [GO:0070946] Definition: Any process that modulates the rate, frequency or extent of neutrophil mediated killing of a gram-positive bacterium, the directed killing of a gram-positive bacterium by a neutrophil. Sources: GOC:add, GOC:mah Subtypes: GO:0070958, positive regulation of neutrophil mediated killing of gram-positive bacterium [GO:0070964]